dihydrolipoamide branched chain acyltransferase activity [GO:0043754] (molecular function) Definition: Catalysis of the reaction: N(6)-[(R)-dihydrolipoyl]-L-lysyl-[protein] + 2-methylpropanoyl-CoA = N(6)-[(R)-S(8)-2-methylpropanoyldihydrolipoyl]-L-lysyl-[protein] + CoA. In addition to transferring the 2-methylpropanoyl group when acting on the oxoacid corresponding with valine, this activity also transfers the 3-methylbutanoyl and S-2-methylbutanoyl groups when acting on the oxo acids corresponding with leucine and isoleucine. Sources: EC:2.3.1.168 Also known as: dihydrolipoamide branched chain transacylase activity, enzyme-dihydrolipoyllysine:2-methylpropanoyl-CoA S-(2-methylpropanoyl)transferase activity, dihydrolipoyllysine-residue (2-methylpropanoyl)transferase activity, 2-methylpropanoyl-CoA:enzyme-6-N-(dihydrolipoyl)lysine:S-(2-methylpropanoyl)transferase activity, 2-methylpropanoyl-CoA:enzyme-N6-(dihydrolipoyl)lysine:S-(2-methylpropanoyl)transferase activity, dihydrolipoyl transacylase activity Relationships: is a type of acyltransferase activity, transferring groups other than amino-acyl groups [GO:0016747]